arginine kinase activity [GO:0004054] (molecular function) Also known as: ATP:L-arginine N-phosphotransferase activity, adenosine 5'-triphosphate-arginine phosphotransferase activity, adenosine 5'-triphosphate:L-arginine, arginine phosphokinase activity Sources: EC:2.7.3.3, RHEA:22940 Definition: Catalysis of the reaction: L-arginine + ATP = N(omega)-phospho-L-arginine + ADP + 2 H+. Relationships: is a type of phosphotransferase activity, nitrogenous group as acceptor [GO:0016775]; is a type of GO:0019202